Asi complex [GO:0097658] (cellular component) Relationships: is a type of nuclear ubiquitin ligase complex [GO:0000152]; is a type of GO:0098796; is part of nuclear inner membrane [GO:0005637] References: PMID:25236469 Sources: GOC:mcc Definition: A nuclear ubiquitin ligase multiprotein complex located in the inner nuclear membrane (INM) that recognizes and ubiquitinates misfolded INM proteins and also some proteins involved in sterol biosynthesis, during ER-associated protein degradation (ERAD). In S. cerevisiae, this complex contains the ubiquitin ligases Asi1p and Asi3p.